{
  "gene_symbol": "ABI1",
  "term_id": "GO:0098858",
  "gene": "UniProtKB:Q8IZP0",
  "term_label": "actin-based cell projection",
  "gene_name": "Abl interactor 1"
}